mRNA processing [GO:0006397] (biological process) Definition: Any process involved in the conversion of a primary mRNA transcript into one or more mature mRNA(s) prior to translation into polypeptide. Regulation: regulated by regulation of mRNA processing [GO:0050684]; positively regulated by positive regulation of mRNA processing [GO:0050685]; negatively regulated by negative regulation of mRNA processing [GO:0050686] Sources: GOC:mah Subtypes: GO:0000398, 7-methylguanosine mRNA capping [GO:0006370], chloroplast mRNA processing [GO:0010239], mRNA 3'-end processing [GO:0031124], GO:0031426, mRNA splicing, via endonucleolytic cleavage and ligation [GO:0070054], mitochondrial mRNA processing [GO:0090615] Also known as: mRNA maturation Relationships: is a type of RNA processing [GO:0006396]; is a type of GO:0016071